{
  "term_id": "GO:0031721",
  "gene": "UniProtKB:P68871",
  "gene_symbol": "HBB",
  "term_label": "hemoglobin alpha binding",
  "gene_name": "Hemoglobin subunit beta"
}